{
  "term_id": "GO:0031640",
  "gene_name": "Histatin-1",
  "gene": "UniProtKB:P15515",
  "term_label": "killing of cells of another organism",
  "gene_symbol": "HTN1"
}